{
  "gene_symbol": "HSPA7",
  "term_label": "protein folding chaperone",
  "gene": "UniProtKB:P48741",
  "term_id": "GO:0044183",
  "gene_name": "Putative heat shock 70 kDa protein 7"
}